{
  "gene_symbol": "DEPDC1",
  "gene_name": "DEP domain-containing protein 1A",
  "term_label": "Unknown molecular function",
  "term_id": "UNKNOWN:0001",
  "gene": "UniProtKB:Q5TB30"
}